negative regulation of dipeptide transport [GO:2000879] (biological process) Subtypes: negative regulation of dipeptide transmembrane transport [GO:2001149] Relationships: is a type of regulation of dipeptide transport [GO:0090089]; is a type of GO:2000877; negatively regulates dipeptide transport [GO:0042938] Sources: GOC:obol Definition: Any process that stops, prevents or reduces the frequency, rate or extent of dipeptide transport.